{
  "term_id": "GO:0030198",
  "term_label": "extracellular matrix organization",
  "gene": "UniProtKB:Q8TE57",
  "gene_symbol": "ADAMTS16",
  "gene_name": "A disintegrin and metalloproteinase with thrombospondin motifs 16"
}